regulation of DNA-templated transcription initiation [GO:2000142] (biological process) Definition: Any process that modulates the frequency, rate or extent of DNA-templated transcription initiation. Subtypes: regulation of transcription initiation by RNA polymerase II [GO:0060260], GO:1903357, negative regulation of DNA-templated transcription initiation [GO:2000143], positive regulation of DNA-templated transcription initiation [GO:2000144] Also known as: regulation of DNA-dependent transcription, initiation, regulation of DNA-templated transcription, initiation, regulation of initiation of DNA-dependent transcription, regulation of transcription initiation, DNA-dependent Relationships: is a type of GO:0006355; regulates DNA-templated transcription initiation [GO:0006352] Sources: GOC:mah, GOC:txnOH